{
  "gene": "UniProtKB:Q16663",
  "gene_name": "C-C motif chemokine 15",
  "gene_symbol": "CCL15",
  "term_label": "extracellular space",
  "term_id": "GO:0005615"
}